cellular response to acid chemical [GO:0071229] (biological process) Definition: Any process that results in a change in state or activity of a cell (in terms of movement, secretion, enzyme production, gene expression, etc.) as a result of a stimulus by the chemical structure of the anion portion of the dissociated acid (rather than the acid acting as a proton donor). The acid chemical may be in gaseous, liquid or solid form. Subtypes: GO:0071230, GO:0071462 Also known as: cellular response to acid, cellular response to acid anion, cellular response to oxoanion Note: This term should be used to describe a response to a specific acid as a chemical. E.g., if a cell were responding to glutamate, then the response would be glutamate-specific; the cell is actually responding to the chemical structure of the anion portion of the dissociated acid. Note that this term is in the subset of terms that should not be used for direct gene product annotation. Instead, select a child term or, if no appropriate child term exists, please request a new term. Direct annotations to this term may be amended during annotation QC. If annotating experiments where an acid is playing a role as a proton donor, please annotate to GO:0071468 'cellular response to acidic pH' instead. Relationships: is a type of response to acid chemical [GO:0001101]; is a type of cellular response to chemical stimulus [GO:0070887] Sources: GOC:go_curators, GOC:mah, Wikipedia:Acid